{
  "term_id": "UNKNOWN:0001",
  "gene": "UniProtKB:Q9BYD5",
  "gene_symbol": "CNFN",
  "gene_name": "Cornifelin",
  "term_label": "Unknown molecular function"
}